{
  "gene_name": "Coiled-coil domain-containing protein 171",
  "gene_symbol": "CCDC171",
  "gene": "UniProtKB:Q6TFL3",
  "term_id": "UNKNOWN:0002",
  "term_label": "Unknown biological process"
}